{
  "term_id": "GO:0019221",
  "gene": "UniProtKB:P78552",
  "gene_name": "Interleukin-13 receptor subunit alpha-1",
  "term_label": "cytokine-mediated signaling pathway",
  "gene_symbol": "IL13RA1"
}